{
  "term_label": "nucleus",
  "term_id": "GO:0005634",
  "gene_name": "Wilms tumor protein 1-interacting protein",
  "gene": "UniProtKB:A6NIX2",
  "gene_symbol": "WTIP"
}